{
  "gene": "UniProtKB:Q96LA9",
  "term_label": "G protein-coupled receptor signaling pathway",
  "gene_symbol": "MRGPRX4",
  "term_id": "GO:0007186",
  "gene_name": "Mas-related G-protein coupled receptor member X4"
}